cell differentiation involved in phenotypic switching [GO:0090679] (biological process) Relationships: is a type of cell differentiation [GO:0030154]; is part of GO:0090677 Definition: A cell differentiation process that is a part of a reversible switch of a cell from one cell type or form to another, at a frequency above the expected frequency for somatic mutations. Sources: GOC:curators Regulation: regulated by regulation of cell differentiation involved in phenotypic switching [GO:1905915]; negatively regulated by negative regulation of cell differentiation involved in phenotypic switching [GO:1905916]; RO_0002213 by positive regulation of cell differentiation involved in phenotypic switching [GO:1905917] Subtypes: GO:1905420